{
  "gene": "UniProtKB:Q14206",
  "gene_symbol": "RCAN2",
  "term_label": "calcium-mediated signaling",
  "term_id": "GO:0019722",
  "gene_name": "Calcipressin-2"
}